{
  "gene_symbol": "EFCC1",
  "gene_name": "EF-hand and coiled-coil domain-containing protein 1",
  "gene": "UniProtKB:Q9HA90",
  "term_label": "Unknown molecular function",
  "term_id": "UNKNOWN:0001"
}